{
  "gene": "UniProtKB:Q9BVW5",
  "term_label": "DNA replication checkpoint signaling",
  "gene_name": "TIMELESS-interacting protein",
  "gene_symbol": "TIPIN",
  "term_id": "GO:0000076"
}